{
  "gene_name": "Phosphatidylinositol 3-kinase C2 domain-containing subunit gamma",
  "gene_symbol": "PIK3C2G",
  "gene": "UniProtKB:O75747",
  "term_id": "GO:0036092",
  "term_label": "phosphatidylinositol-3-phosphate biosynthetic process"
}